{
  "gene_name": "Cadherin EGF LAG seven-pass G-type receptor 3",
  "gene_symbol": "CELSR3",
  "gene": "UniProtKB:Q9NYQ7",
  "term_id": "GO:0044331",
  "term_label": "cell-cell adhesion mediated by cadherin"
}